{
  "gene_symbol": "PARN",
  "term_id": "GO:0003723",
  "gene_name": "Poly(A)-specific ribonuclease PARN",
  "term_label": "RNA binding",
  "gene": "UniProtKB:O95453"
}